{
  "gene_name": "Transient receptor potential cation channel subfamily M member 7",
  "term_id": "GO:0005886",
  "term_label": "plasma membrane",
  "gene_symbol": "TRPM7",
  "gene": "UniProtKB:Q96QT4"
}